peptidyl-proline hydroxylation to 3-hydroxy-L-proline [GO:0018400] (biological process) Relationships: is a type of modified amino acid metabolic process [GO:0006575]; is a type of GO:0019511; is_a L-amino acid metabolic process [GO:0170033]; is a type of GO:0170041 Definition: The modification of peptidyl-proline to form 3-hydroxy-L-proline; catalyzed by procollagen-proline 3-dioxygenase. Note: See also the molecular function term 'procollagen-proline 3-dioxygenase activity ; GO:0019797'. Sources: RESID:AA0029